{
  "gene": "UniProtKB:Q9GZX9",
  "term_id": "GO:0005615",
  "gene_symbol": "TWSG1",
  "term_label": "extracellular space",
  "gene_name": "Twisted gastrulation protein homolog 1"
}